{
  "gene_symbol": "A1CF",
  "gene_name": "APOBEC1 complementation factor",
  "gene": "UniProtKB:Q9NQ94",
  "term_id": "GO:0005634",
  "term_label": "nucleus"
}